positive regulation of calcium ion transport into cytosol involved in cellular response to salt stress [GO:1901199] (biological process) Definition: Any positive regulation of calcium ion transport into cytosol that is involved in cellular response to salt stress. Relationships: is a type of positive regulation of calcium ion transport into cytosol [GO:0010524]; is part of cellular response to salt stress [GO:0071472] Also known as: positive regulation of calcium ion transport into cytosol involved in cellular response to ionic osmotic stress, positive regulation of calcium ion transport into cytosol involved in cellular salinity response Sources: GOC:TermGenie